ABC-type glycine betaine transporter activity [GO:0031459] (molecular function) Definition: Catalysis of the reaction: ATP + H2O + glycine betaine(out) = ADP + phosphate + glycine betaine(in). Sources: GOC:mlg, RHEA:32783 Also known as: ATP-dependent glycine betaine transporter activity, N-trimethylglycine-transporting ATPase activity, glycine betaine ABC transporter, ATPase-coupled glycine betaine transporter activity, glycine betaine-transporting ATPase activity Relationships: is_a amino-acid betaine transmembrane transporter activity [GO:0015199]; is_a ABC-type quaternary ammonium compound transporting activity [GO:0015418]; is part of glycine betaine transport [GO:0031460]